(S)-limonene 6-monooxygenase activity [GO:0018675] (molecular function) Relationships: is a type of oxidoreductase activity, acting on paired donors, with incorporation or reduction of molecular oxygen, reduced flavin or flavoprotein as one donor, and incorporation of one atom of oxygen [GO:0016712]; is a type of GO:0019113 Sources: RHEA:17945 Definition: Catalysis of the reaction: (4S)-limonene + O2 + reduced [NADPH--hemoprotein reductase] = (1S,5R)-carveol + H+ + H2O + oxidized [NADPH--hemoprotein reductase]. Also known as: (-)-limonene 6-monooxygenase activity, limonene 6-hydroxylase activity, (-)-limonene 6-hydroxylase activity, (-)-limonene,NADPH:oxygen oxidoreductase (6-hydroxylating) activity, (S)-limonene,NADPH:oxygen oxidoreductase (6-hydroxylating)